{
  "term_label": "Unknown cellular component",
  "gene_name": "Uncharacterized protein C2orf50",
  "gene": "UniProtKB:Q96LR7",
  "gene_symbol": "C2orf50",
  "term_id": "UNKNOWN:0003"
}